{
  "gene_name": "Zinc finger and SCAN domain-containing protein 23",
  "gene": "UniProtKB:Q3MJ62",
  "term_label": "DNA-binding transcription factor activity, RNA polymerase II-specific",
  "gene_symbol": "ZSCAN23",
  "term_id": "GO:0000981"
}